regulation of tRNA methylation [GO:0110002] (biological process) Definition: Any process that modulates the frequency, rate or extent of the chemical reactions and pathways involving tRNA methylation. Subtypes: regulation of tRNA C5-cytosine methylation [GO:0110003], positive regulation of tRNA methylation [GO:0110004] References: PMID:23074192 Sources: GOC:vw Relationships: is a type of regulation of tRNA processing [GO:2000235]; regulates tRNA methylation [GO:0030488]